{
  "term_label": "collagen metabolic process",
  "gene_symbol": "P3H2",
  "term_id": "GO:0032963",
  "gene_name": "Prolyl 3-hydroxylase 2",
  "gene": "UniProtKB:Q8IVL5"
}